{
  "term_id": "GO:0034976",
  "gene": "UniProtKB:P30101",
  "gene_name": "Protein disulfide-isomerase A3",
  "gene_symbol": "PDIA3",
  "term_label": "response to endoplasmic reticulum stress"
}